{
  "gene": "UniProtKB:O75747",
  "term_label": "cytoplasm",
  "term_id": "GO:0005737",
  "gene_symbol": "PIK3C2G",
  "gene_name": "Phosphatidylinositol 3-kinase C2 domain-containing subunit gamma"
}